3-hydroxyphenyl propanoate transmembrane transporter activity [GO:0015551] (molecular function) Definition: Enables the transfer of 3-hydroxyphenyl propanoate from one side of a membrane to the other. Sources: GOC:ai Also known as: 3-hydroxyphenyl propionate transmembrane transporter activity Relationships: is a type of GO:0022857; is part of 3-hydroxyphenyl propanoate transport [GO:0015731] Subtypes: 3-hydroxyphenyl propionate:proton symporter activity [GO:0015540]